negative regulation of defense response to virus by host [GO:0050689] (biological process) Sources: GOC:ai, GOC:dph, GOC:tb Definition: Any host process that results in the inhibition of antiviral immune response mechanisms, thereby facilitating viral replication. The host is defined as the larger of the organisms involved in a symbiotic interaction. Also known as: down regulation of antiviral response by host, down-regulation of antiviral response by host, downregulation of antiviral response by host, negative regulation by host of antiviral response, negative regulation of antiviral response by host, inhibition of antiviral response by host Relationships: is_a GO:0050687; is a type of GO:0050691